{
  "gene_name": "Alpha-1-antichymotrypsin",
  "term_label": "extracellular space",
  "gene_symbol": "SERPINA3",
  "term_id": "GO:0005615",
  "gene": "UniProtKB:P01011"
}